{
  "gene_name": "CUE domain-containing protein 2",
  "gene": "UniProtKB:Q9H467",
  "gene_symbol": "CUEDC2",
  "term_id": "UNKNOWN:0001",
  "term_label": "Unknown molecular function"
}